blasticidin S catabolic process [GO:1905265] (biological process) Definition: The chemical reactions and pathways resulting in the breakdown of blasticidin S. References: PMID:23874663 Sources: GOC:TermGenie, GOC:pr, GO_REF:0000068, Wikipedia:Blasticidin_S Also known as: blasticidin S breakdown, blasticidin S catabolism, blasticidin S degradation Relationships: is a type of GO:0046135